{
  "term_label": "phosphoric diester hydrolase activity",
  "gene_symbol": "PLCXD1",
  "gene": "UniProtKB:Q9NUJ7",
  "gene_name": "PI-PLC X domain-containing protein 1",
  "term_id": "GO:0008081"
}